calcium-ion regulated exocytosis [GO:0017156] (biological process) Subtypes: GO:0048791, cortical granule exocytosis [GO:0060471], GO:0060478, zymogen granule exocytosis [GO:0070625], dense core granule exocytosis [GO:1990504], calcium ion regulated lysosome exocytosis [GO:1990927] Sources: GOC:go_curators Relationships: is a type of regulated exocytosis [GO:0045055] Definition: The release of intracellular molecules (e.g. hormones, matrix proteins) contained within a membrane-bounded vesicle by fusion of the vesicle with the plasma membrane of a cell, induced by a rise in cytosolic calcium-ion levels. Also known as: calcium ion-dependent exocytosis Regulation: regulated by regulation of calcium ion-dependent exocytosis [GO:0017158]; negatively regulated by negative regulation of calcium ion-dependent exocytosis [GO:0045955]; positively regulated by GO:0045956 Note: Note that the calcium regulated exocytosis pathway can be leaky: some level of exocytosis via this pathway occurs spontaneously. This phenomenon underlies spontaneous neurotransmitter release from presynapses. This phenomenon is distinct from the unregulated, calcium independent exocytosis pathway.